{
  "gene_symbol": "AHCTF1",
  "gene_name": "Protein ELYS",
  "gene": "UniProtKB:Q8WYP5",
  "term_label": "Unknown molecular function",
  "term_id": "UNKNOWN:0001"
}